{
  "gene_name": "Small ribosomal subunit protein uS2B",
  "term_label": "structural constituent of ribosome",
  "term_id": "GO:0003735",
  "gene_symbol": "RPSA2",
  "gene": "UniProtKB:A0A8I5KQE6"
}